{
  "gene_name": "WD repeat-containing protein 70",
  "gene": "UniProtKB:Q9NW82",
  "gene_symbol": "WDR70",
  "term_label": "Unknown molecular function",
  "term_id": "UNKNOWN:0001"
}